{
  "gene_name": "Cone cGMP-specific 3',5'-cyclic phosphodiesterase subunit alpha'",
  "term_label": "3',5'-cyclic-GMP phosphodiesterase activity",
  "term_id": "GO:0047555",
  "gene": "UniProtKB:P51160",
  "gene_symbol": "PDE6C"
}